2,5-dioxopiperazine hydrolase activity [GO:0047532] (molecular function) Also known as: 2,5-dioxopiperazine amidohydrolase activity, cyclo(Gly-Gly) hydrolase activity, cyclo(glycylglycine) hydrolase activity Relationships: is a type of GO:0016812 Sources: EC:3.5.2.13, RHEA:21808 Definition: Catalysis of the reaction: 2,5-dioxopiperazine + H2O = glycylglycine.